regulation of establishment of blood-brain barrier [GO:0090210] (biological process) Sources: GOC:dph, GOC:tb Subtypes: positive regulation of establishment of blood-brain barrier [GO:0090211], GO:0090212 Definition: Any process that modulates the rate, frequency or extent of the establishment of the blood-brain barrier, a selectively permeable structural and functional barrier that exists between the capillaries and the brain. Relationships: is a type of regulation of cell development [GO:0060284]; regulates establishment of blood-brain barrier [GO:0060856] Also known as: regulation of establishment of BBB